{
  "gene_symbol": "DLG3",
  "gene": "UniProtKB:Q92796",
  "term_id": "GO:0045197",
  "term_label": "establishment or maintenance of epithelial cell apical/basal polarity",
  "gene_name": "Disks large homolog 3"
}